glycerol-3-phosphate dehydrogenase (FAD) complex [GO:0009331] (cellular component) Relationships: is_a GO:1990204; is part of GO:0005737 Also known as: glycerol-3-phosphate dehydrogenase complex, aerobic glycerol 3-phosphate dehydrogenase, anaerobic glycerol-3-phosphate dehydrogenase References: PMID:18296637, PMID:3286606, PMID:7576488 Definition: An enzyme complex that catalyzes the oxidation of sn-glycerol 3-phosphate to dihydroxyacetone phosphate, with concurrent reduction of flavin adenine dinucleotide (FAD) to FADH2. In E. coli, the complex is either a GlpA-GlpB-GlpC heterotrimer that functions in anaerobic conditions, or a GlpD homodimer that functions in aerobic conditions.